{
  "gene_name": "Mitochondrial import inner membrane translocase subunit TIM16",
  "term_id": "GO:0030150",
  "term_label": "protein import into mitochondrial matrix",
  "gene_symbol": "PAM16",
  "gene": "UniProtKB:Q9Y3D7"
}